10-formyltetrahydrofolate catabolic process [GO:0009258] (biological process) Definition: The chemical reactions and pathways resulting in the breakdown of 10-formyltetrahydrofolate, the formylated derivative of tetrahydrofolate. Sources: GOC:ai Relationships: is a type of 10-formyltetrahydrofolate metabolic process [GO:0009256]; is a type of GO:0009397; is a type of dicarboxylic acid catabolic process [GO:0043649] Also known as: 10-formyl-THF catabolic process, 10-formyl-THF catabolism, 10-formyltetrahydrofolate breakdown, 10-formyltetrahydrofolate catabolism, 10-formyltetrahydrofolate degradation